{
  "gene": "UniProtKB:O75143",
  "gene_name": "Autophagy-related protein 13",
  "term_label": "Atg1/ULK1 kinase complex",
  "term_id": "GO:1990316",
  "gene_symbol": "ATG13"
}